{
  "gene": "UniProtKB:Q06730",
  "term_id": "GO:0005634",
  "term_label": "nucleus",
  "gene_symbol": "ZNF33A",
  "gene_name": "Zinc finger protein 33A"
}